symbiont-mediated-mediated suppression of host tetherin activity [GO:0039587] (biological process) Also known as: inhibition of host BST2/Tetherin by virus, suppression by virus of host tetherin activity, evasion of suppression of viral release by host via inhibition of host tetherin activity References: PMID:22493439 Definition: Any process in which a symbiont stops, prevents, or reduces the activity of host tetherin activity. Tetherin (also known as BST2) is an alpha interferon-inducible cellular factor that impairs the release of many enveloped viruses. By blocking tetherin activity, many viruses circumvent its antiviral effects. Relationships: is a type of GO:0052031